{
  "term_id": "GO:0045202",
  "gene_name": "Glypican-2",
  "term_label": "synapse",
  "gene": "UniProtKB:Q8N158",
  "gene_symbol": "GPC2"
}